{
  "term_label": "phototransduction",
  "gene_symbol": "OPN1MW3",
  "gene_name": "Medium-wave-sensitive opsin 3",
  "term_id": "GO:0007602",
  "gene": "UniProtKB:P0DN78"
}